extension of leading cell process to pial surface [GO:0021803] (biological process) References: PMID:12626695 Sources: GOC:cls, GOC:dgh, GOC:dph, GOC:jid, GO_REF:0000021 Relationships: is_a plasma membrane bounded cell projection assembly [GO:0120031]; is part of somal translocation [GO:0021802] Definition: The extension of a long process to the pial surface as a cell leaves the ventricular zone.